{
  "term_label": "Unknown biological process",
  "term_id": "UNKNOWN:0002",
  "gene_symbol": "ODAD2",
  "gene": "UniProtKB:Q5T2S8",
  "gene_name": "Outer dynein arm-docking complex subunit 2"
}